urate transport [GO:0015747] (biological process) Definition: The directed movement of urate into, out of or within a cell, or between cells, by means of some agent such as a transporter or pore. Sources: GOC:krc Also known as: urate transmembrane transport, uric acid transport Relationships: is a type of organic anion transport [GO:0015711]; is a type of nitrogen compound transport [GO:0071705]